{
  "term_id": "GO:0006256",
  "gene": "UniProtKB:Q9Y227",
  "gene_name": "Ectonucleoside triphosphate diphosphohydrolase 4",
  "term_label": "UDP catabolic process",
  "gene_symbol": "ENTPD4"
}